{
  "gene_name": "Tyrosine-protein kinase Lck",
  "term_id": "GO:0005886",
  "gene": "UniProtKB:P06239",
  "gene_symbol": "LCK",
  "term_label": "plasma membrane"
}